{
  "term_label": "structural constituent of skin epidermis",
  "gene_symbol": "KRT13",
  "gene_name": "Keratin, type I cytoskeletal 13",
  "gene": "UniProtKB:P13646",
  "term_id": "GO:0030280"
}